{
  "gene_name": "17-beta-hydroxysteroid dehydrogenase type 1",
  "gene_symbol": "HSD17B1",
  "term_id": "GO:0006703",
  "term_label": "estrogen biosynthetic process",
  "gene": "UniProtKB:P14061"
}